{
  "term_label": "Unknown biological process",
  "term_id": "UNKNOWN:0002",
  "gene": "UniProtKB:Q5RHP9",
  "gene_name": "Glutamate-rich protein 3",
  "gene_symbol": "ERICH3"
}